{
  "gene_name": "E3 SUMO-protein ligase CBX4",
  "term_id": "GO:0061665",
  "gene_symbol": "CBX4",
  "gene": "UniProtKB:O00257",
  "term_label": "SUMO ligase activity"
}